macrophage migration inhibitory factor signaling pathway [GO:0035691] (biological process) Also known as: MIF signaling pathway, macrophage migration inhibitory factor signalling pathway References: PMID:12782713, PMID:19413900 Sources: GOC:BHF, GOC:signaling Definition: The series of molecular signals initiated by macrophage migration inhibitory factor binding to its receptor on the surface of a target cell, and ending with the regulation of a downstream cellular process, e.g. transcription. Regulation: regulated by GO:2000446; negatively regulated by GO:2000447; positively regulated by positive regulation of macrophage migration inhibitory factor signaling pathway [GO:2000448] Relationships: is a type of cytokine-mediated signaling pathway [GO:0019221]